{
  "gene_name": "Fms-related tyrosine kinase 3 ligand",
  "gene_symbol": "FLT3LG",
  "term_label": "positive regulation of cell population proliferation",
  "gene": "UniProtKB:P49771",
  "term_id": "GO:0008284"
}